uredospore formation [GO:0075251] (biological process) Regulation: RO_0002211 by regulation of uredospore formation [GO:0075252]; positively regulated by positive regulation of uredospore formation [GO:0075253]; negatively regulated by negative regulation of uredospore formation [GO:0075254] Relationships: is a type of asexual sporulation resulting in formation of a cellular spore [GO:0043936] Sources: GOC:pamgo_curators Also known as: urediniospore formation, ureidospore formation Definition: The process which specific outcome is the formation of an asexual, dikaryotic, often rusty-colored spore, produced in a structure called a uredinium; mostly found in the rust fungus.